{
  "term_id": "GO:0016593",
  "gene_symbol": "PAF1",
  "term_label": "Cdc73/Paf1 complex",
  "gene": "UniProtKB:Q8N7H5",
  "gene_name": "RNA polymerase II-associated factor 1 homolog"
}